{
  "gene_symbol": "SHOC2",
  "term_label": "nerve growth factor signaling pathway",
  "gene": "UniProtKB:Q9UQ13",
  "gene_name": "Leucine-rich repeat protein SHOC-2",
  "term_id": "GO:0038180"
}